{
  "gene": "UniProtKB:Q14005",
  "term_label": "cytokine-mediated signaling pathway",
  "gene_name": "Pro-interleukin-16",
  "gene_symbol": "IL16",
  "term_id": "GO:0019221"
}